{
  "gene": "UniProtKB:Q9ULD0",
  "term_id": "GO:0045252",
  "gene_symbol": "OGDHL",
  "term_label": "oxoglutarate dehydrogenase complex",
  "gene_name": "2-oxoglutarate dehydrogenase-like, mitochondrial"
}